{
  "gene_name": "Putative elongation factor 1-delta-like protein",
  "term_label": "Unknown biological process",
  "term_id": "UNKNOWN:0002",
  "gene": "UniProtKB:Q658K8",
  "gene_symbol": "EEF1DP3"
}